{
  "gene_name": "RANBP2-like and GRIP domain-containing protein 2",
  "gene": "UniProtKB:P0DJD1",
  "gene_symbol": "RGPD2",
  "term_label": "nuclear export",
  "term_id": "GO:0051168"
}